{
  "gene": "UniProtKB:Q9Y2X3",
  "term_label": "snoRNA binding",
  "gene_symbol": "NOP58",
  "gene_name": "Nucleolar protein 58",
  "term_id": "GO:0030515"
}